{
  "gene_symbol": "C1QBP",
  "gene": "UniProtKB:Q07021",
  "term_id": "GO:0009986",
  "term_label": "cell surface",
  "gene_name": "Complement component 1 Q subcomponent-binding protein, mitochondrial"
}